{
  "term_id": "GO:0043565",
  "gene": "UniProtKB:P55895",
  "gene_symbol": "RAG2",
  "gene_name": "V(D)J recombination-activating protein 2",
  "term_label": "sequence-specific DNA binding"
}